{
  "term_id": "GO:0006338",
  "term_label": "chromatin remodeling",
  "gene": "UniProtKB:Q92833",
  "gene_name": "Protein Jumonji",
  "gene_symbol": "JARID2"
}